{
  "term_label": "L-glutamate transmembrane transporter activity",
  "gene_name": "Vesicular glutamate transporter 3",
  "term_id": "GO:0005313",
  "gene": "UniProtKB:Q8NDX2",
  "gene_symbol": "SLC17A8"
}